{
  "term_label": "endoplasmic reticulum-Golgi intermediate compartment",
  "gene_symbol": "ERP44",
  "term_id": "GO:0005793",
  "gene_name": "Endoplasmic reticulum resident protein 44",
  "gene": "UniProtKB:Q9BS26"
}